regulation of spermidine biosynthetic process [GO:1901304] (biological process) Sources: GOC:TermGenie, GOC:pm Also known as: regulation of spermidine anabolism, regulation of spermidine biosynthesis, regulation of spermidine formation, regulation of spermidine synthesis Definition: Any process that modulates the frequency, rate or extent of spermidine biosynthetic process. Relationships: is_a GO:0010967; regulates GO:0008295 Subtypes: negative regulation of spermidine biosynthetic process [GO:1901305], positive regulation of spermidine biosynthetic process [GO:1901307]